{
  "gene_symbol": "MAGED2",
  "gene_name": "Melanoma-associated antigen D2",
  "gene": "UniProtKB:Q9UNF1",
  "term_id": "GO:0000122",
  "term_label": "negative regulation of transcription by RNA polymerase II"
}